positive regulation of translation in response to stress [GO:0032056] (biological process) Definition: Any process that activates or increases the frequency, rate or extent of translation as a result of a stimulus indicating the organism is under stress. Sources: GOC:mah Also known as: up regulation of translation in response to stress, up-regulation of translation in response to stress, upregulation of translation in response to stress, activation of translation in response to stress, stimulation of translation in response to stress Relationships: is a type of regulation of translation in response to stress [GO:0043555]; is a type of positive regulation of translation [GO:0045727] Subtypes: positive regulation of mitochondrial translation in response to stress [GO:0010892], positive regulation of translation in response to osmotic stress [GO:0032062], GO:0032939, GO:0036493, positive regulation of translational initiation in response to starvation [GO:0071264]